autophagosome membrane docking [GO:0016240] (biological process) Relationships: is a type of GO:0140056; is part of autophagosome maturation [GO:0097352] Also known as: autophagic vacuole docking Definition: The initial attachment of an autophagosome membrane to a target membrane, mediated by proteins protruding from the membrane of the vesicle and the target membrane. Docking requires only that the two membranes come close enough for these proteins to interact and adhere. Sources: GOC:autophagy, GOC:mah